{
  "gene": "UniProtKB:Q9QC07",
  "term_id": "UNKNOWN:0002",
  "term_label": "Unknown biological process",
  "gene_name": "Endogenous retrovirus group K member 18 Pol protein",
  "gene_symbol": "ERVK-18"
}